{
  "gene": "UniProtKB:Q8NGQ5",
  "term_label": "odorant binding",
  "gene_symbol": "OR9Q1",
  "term_id": "GO:0005549",
  "gene_name": "Olfactory receptor 9Q1"
}